L-idonate transmembrane transporter activity [GO:0015568] (molecular function) Definition: Enables the transfer of L-idonate from one side of a membrane to the other. L-idonate is an aldonic acid derived from L-idose, an aldohexose which is epimeric with D-glucose. Sources: GOC:ai Relationships: is a type of monocarboxylic acid transmembrane transporter activity [GO:0008028]; is a type of carbohydrate transmembrane transporter activity [GO:0015144]; is a type of aldonate transmembrane transporter activity [GO:0042879]; is part of L-idonate transmembrane transport [GO:0015726] Also known as: L-idonate/D-gluconate:hydrogen symporter activity